NFAT protein binding [GO:0051525] (molecular function) Also known as: NFAT binding, nuclear factor of activated T cell protein binding, NFAT1 protein binding, NFAT2 protein binding, NFAT3 protein binding, NFAT4 protein binding, NFAT5 protein binding, NFATc binding, NFATc1 binding, NFATc2 binding, NFATc3 binding, NFATc4 binding, NFATp binding, NFATx binding, non-calcium-regulated NFAT protein binding Relationships: is a type of RNA polymerase II-specific DNA-binding transcription factor binding [GO:0061629] Definition: Binding to NFAT (nuclear factor of activated T cells) proteins, a family of transcription factors. NFAT proteins have crucial roles in the development and function of the immune system. References: PMID:15928679